4-phosphoerythronate dehydrogenase activity [GO:0033711] (molecular function) Relationships: is a type of oxidoreductase activity, acting on the CH-OH group of donors, NAD or NADP as acceptor [GO:0016616] Also known as: 4-O-phosphoerythronate dehydrogenase activity, 4-phospho-D-erythronate:NAD+ 2-oxidoreductase activity, 4PE dehydrogenase activity, PdxB, PdxB 4PE dehydrogenase activity, erythronate-4-phosphate dehydrogenase activity Definition: Catalysis of the reaction: 4-phospho-D-erythronate + NAD+ = (R)-3-hydroxy-2-oxo-4-phosphonooxybutanoate + H+ + NADH. Sources: EC:1.1.1.290, RHEA:18829